{
  "term_id": "GO:0045088",
  "gene_name": "Deoxynucleoside triphosphate triphosphohydrolase SAMHD1",
  "term_label": "regulation of innate immune response",
  "gene_symbol": "SAMHD1",
  "gene": "UniProtKB:Q9Y3Z3"
}